intestinal hexose absorption [GO:0106001] (biological process) Subtypes: intestinal D-glucose absorption [GO:0001951] Relationships: is a type of intestinal absorption [GO:0050892] Definition: Uptake of hexoses, notably D-glucose, fructose, and galactose, into the blood by absorption from the small intestine. Sources: GOC:hjd